{
  "gene": "UniProtKB:Q5M9N0",
  "term_label": "Unknown molecular function",
  "gene_symbol": "CCDC158",
  "term_id": "UNKNOWN:0001",
  "gene_name": "Coiled-coil domain-containing protein 158"
}